{
  "gene_symbol": "SCARB2",
  "term_id": "GO:0005886",
  "gene": "UniProtKB:Q14108",
  "gene_name": "Lysosome membrane protein 2",
  "term_label": "plasma membrane"
}